glycerol-1-phosphate dehydrogenase (NAD+) activity [GO:0106357] (molecular function) Definition: Catalysis of the reaction: NAD+ + sn-glycerol 1-phosphate = dihydroxyacetone phosphate + H+ + NADH. Also known as: glycerol-1-phosphate dehydrogenase [NAD+] activity Relationships: is a type of glycerol-1-phosphate dehydrogenase [NAD(P)+] activity [GO:0050492] Sources: RHEA:21412